{
  "term_label": "extracellular space",
  "gene": "UniProtKB:Q96S42",
  "term_id": "GO:0005615",
  "gene_symbol": "NODAL",
  "gene_name": "Nodal homolog"
}